{
  "gene": "UniProtKB:Q15651",
  "term_id": "GO:0003682",
  "term_label": "chromatin binding",
  "gene_symbol": "HMGN3",
  "gene_name": "High mobility group nucleosome-binding domain-containing protein 3"
}